{
  "gene": "UniProtKB:O43166",
  "gene_name": "Signal-induced proliferation-associated 1-like protein 1",
  "gene_symbol": "SIPA1L1",
  "term_id": "GO:0061001",
  "term_label": "regulation of dendritic spine morphogenesis"
}